{
  "gene": "UniProtKB:Q9NX02",
  "gene_name": "NACHT, LRR and PYD domains-containing protein 2",
  "term_label": "cytoplasm",
  "term_id": "GO:0005737",
  "gene_symbol": "NLRP2"
}